cortical microtubule plus-end [GO:1903754] (cellular component) Sources: GOC:TermGenie, GOC:vw, GO_REF:0000064 Definition: The plus-end of a cortical microtubule. Relationships: is a type of GO:1904511; is part of cortical microtubule [GO:0055028] Also known as: cortical microtubule plus end